{
  "gene_name": "Uncharacterized protein KIAA0513",
  "gene": "UniProtKB:O60268",
  "term_id": "UNKNOWN:0003",
  "gene_symbol": "KIAA0513",
  "term_label": "Unknown cellular component"
}